{
  "term_id": "GO:0005634",
  "gene": "UniProtKB:Q9Y6R6",
  "term_label": "nucleus",
  "gene_symbol": "ZNF780B",
  "gene_name": "Zinc finger protein 780B"
}